{
  "term_label": "RNA binding",
  "gene": "UniProtKB:Q9NR56",
  "gene_symbol": "MBNL1",
  "gene_name": "Muscleblind-like protein 1",
  "term_id": "GO:0003723"
}